{
  "gene": "UniProtKB:Q9NX70",
  "term_label": "regulation of transcription by RNA polymerase II",
  "term_id": "GO:0006357",
  "gene_name": "Mediator of RNA polymerase II transcription subunit 29",
  "gene_symbol": "MED29"
}